negative regulation of iodide transport [GO:1904202] (biological process) Relationships: is a type of GO:1903792; is a type of regulation of iodide transport [GO:1904201]; negatively regulates GO:0015705 Definition: Any process that stops, prevents or reduces the frequency, rate or extent of iodide transport. Subtypes: negative regulation of iodide transmembrane transport [GO:1904213] Also known as: down regulation of iodide transport, down-regulation of iodide transport, downregulation of iodide transport, inhibition of iodide transport References: PMID:20392814 Sources: GOC:TermGenie, GO_REF:0000058